{
  "term_id": "GO:0001786",
  "gene_symbol": "ANXA13",
  "term_label": "phosphatidylserine binding",
  "gene_name": "Annexin A13",
  "gene": "UniProtKB:P27216"
}